{
  "gene_name": "Neurotrophin-4",
  "term_id": "GO:0050804",
  "term_label": "modulation of chemical synaptic transmission",
  "gene": "UniProtKB:P34130",
  "gene_symbol": "NTF4"
}